negative regulation of androst-4-ene-3,17-dione biosynthetic process [GO:1903455] (biological process) Relationships: is a type of negative regulation of steroid biosynthetic process [GO:0010894]; is a type of negative regulation of small molecule metabolic process [GO:0062014]; is a type of regulation of androst-4-ene-3,17-dione biosynthetic process [GO:1903454]; negatively regulates androst-4-ene-3,17-dione biosynthetic process [GO:1903449] References: PMID:24399684 Sources: GOC:TermGenie, GOC:mr, GO_REF:0000058 Definition: Any process that stops, prevents or reduces the frequency, rate or extent of androst-4-ene-3,17-dione biosynthetic process. Also known as: down regulation of androst-4-ene-3,17-dione anabolism, down regulation of androst-4-ene-3,17-dione biosynthesis, down regulation of androst-4-ene-3,17-dione biosynthetic process, down regulation of androst-4-ene-3,17-dione formation, down regulation of androst-4-ene-3,17-dione synthesis, down regulation of androstenedione biosynthetic process, down-regulation of androst-4-ene-3,17-dione anabolism, down-regulation of androst-4-ene-3,17-dione biosynthesis, down-regulation of androst-4-ene-3,17-dione biosynthetic process, down-regulation of androst-4-ene-3,17-dione formation, down-regulation of androst-4-ene-3,17-dione synthesis, down-regulation of androstenedione biosynthetic process, downregulation of androst-4-ene-3,17-dione anabolism, downregulation of androst-4-ene-3,17-dione biosynthesis, downregulation of androst-4-ene-3,17-dione biosynthetic process, downregulation of androst-4-ene-3,17-dione formation, downregulation of androst-4-ene-3,17-dione synthesis, downregulation of androstenedione biosynthetic process, negative regulation of androst-4-ene-3,17-dione anabolism, negative regulation of androst-4-ene-3,17-dione biosynthesis, negative regulation of androst-4-ene-3,17-dione formation, negative regulation of androst-4-ene-3,17-dione synthesis, negative regulation of androstenedione biosynthetic process, inhibition of androst-4-ene-3,17-dione anabolism, inhibition of androst-4-ene-3,17-dione biosynthesis, inhibition of androst-4-ene-3,17-dione biosynthetic process, inhibition of androst-4-ene-3,17-dione formation, inhibition of androst-4-ene-3,17-dione synthesis, inhibition of androstenedione